{
  "gene": "UniProtKB:Q13207",
  "term_id": "GO:0001708",
  "term_label": "cell fate specification",
  "gene_symbol": "TBX2",
  "gene_name": "T-box transcription factor TBX2"
}